regulation of translational elongation [GO:0006448] (biological process) Relationships: is_a regulation of translation [GO:0006417]; regulates translational elongation [GO:0006414] Definition: Any process that modulates the frequency, rate, extent or accuracy of translational elongation. Sources: GOC:go_curators Subtypes: GO:0045900, GO:0045901, regulation of cytoplasmic translational elongation [GO:1900247], regulation of selenocysteine incorporation [GO:1904569], GO:1905082, regulation of translational frameshifting [GO:2001124]